{
  "term_id": "GO:0055085",
  "gene_name": "Electrogenic sodium bicarbonate cotransporter 4",
  "gene_symbol": "SLC4A5",
  "gene": "UniProtKB:Q9BY07",
  "term_label": "transmembrane transport"
}